{
  "gene_name": "Gamma-aminobutyric acid receptor subunit alpha-1",
  "gene": "UniProtKB:P14867",
  "term_label": "chloride transmembrane transport",
  "term_id": "GO:1902476",
  "gene_symbol": "GABRA1"
}